double-strand break repair via homologous recombination [GO:0000724] (biological process) Definition: The error-free repair of a double-strand break in DNA in which the broken DNA molecule is repaired using homologous sequences. A strand in the broken DNA searches for a homologous region in an intact chromosome to serve as the template for DNA synthesis. The restoration of two intact DNA molecules results in the exchange, reciprocal or nonreciprocal, of genetic material between the intact DNA molecule and the broken DNA molecule. Also known as: HDR, HRR, Rad51-dependent recombinational repair, Rhp51-dependent recombinational repair, homologous recombinational repair, homology-directed repair Regulation: regulated by regulation of double-strand break repair via homologous recombination [GO:0010569]; positively regulated by positive regulation of double-strand break repair via homologous recombination [GO:1905168]; negatively regulated by negative regulation of double-strand break repair via homologous recombination [GO:2000042] Relationships: is a type of recombinational repair [GO:0000725]; is_a double-strand break repair [GO:0006302] Subtypes: double-strand break repair via break-induced replication [GO:0000727], double-strand break repair via synthesis-dependent strand annealing [GO:0045003], double-strand break repair via transcription-associated homologous recombination [GO:0106400], replication-born double-strand break repair via sister chromatid exchange [GO:1990414] References: PMID:10357855 Sources: GOC:elh